{
  "gene": "UniProtKB:P15260",
  "gene_symbol": "IFNGR1",
  "gene_name": "Interferon gamma receptor 1",
  "term_label": "plasma membrane",
  "term_id": "GO:0005886"
}